mitochondrion-endoplasmic reticulum membrane tethering [GO:1990456] (biological process) References: PMID:19556461, PMID:27875684 Also known as: mitochondrion-ER attachment, mitochondrion-ER membrane tethering, mitochondrion-ER tethering, mitochondrion-endoplasmic reticulum attachment, mitochondrion-endoplasmic reticulum tethering Relationships: is a type of GO:0016043; is a type of organelle localization by membrane tethering [GO:0140056] Definition: The attachment of a mitochondrion and an endoplasmic reticulum via molecular tethers that physically bridge their respective membranes and attach them to each other. The tethering may facilitate exchange of metabolites between the organelles.